{
  "term_id": "UNKNOWN:0002",
  "gene_symbol": "ZFAND3",
  "term_label": "Unknown biological process",
  "gene_name": "AN1-type zinc finger protein 3",
  "gene": "UniProtKB:Q9H8U3"
}